{
  "gene_name": "Kelch-like protein 22",
  "gene_symbol": "KLHL22",
  "term_id": "GO:1904263",
  "term_label": "positive regulation of TORC1 signaling",
  "gene": "UniProtKB:Q53GT1"
}